organelle membrane [GO:0031090] (cellular component) Subtypes: endoplasmic reticulum membrane [GO:0005789], vesicle membrane [GO:0012506], organelle inner membrane [GO:0019866], symbiont-containing vacuole membrane [GO:0020005], nuclear membrane [GO:0031965], GO:0031966, GO:0032580, trans-Golgi network membrane [GO:0032588], GO:0033016, plastid membrane [GO:0042170], photoreceptor disc membrane [GO:0097381], bounding membrane of organelle [GO:0098588], magnetosome membrane [GO:0110146], perinuclear endoplasmic reticulum membrane [GO:1990578] Also known as: intracellular membrane Sources: GOC:dos, GOC:mah Relationships: is_a membrane [GO:0016020]; is part of membrane-bounded organelle [GO:0043227] Definition: A membrane that is one of the two lipid bilayers of an organelle envelope or the outermost membrane of single membrane bound organelle.